{
  "gene_symbol": "TUBA1A",
  "term_id": "GO:0000226",
  "gene": "UniProtKB:Q71U36",
  "gene_name": "Tubulin alpha-1A chain",
  "term_label": "microtubule cytoskeleton organization"
}